{
  "gene_symbol": "TSSC4",
  "term_label": "molecular sequestering activity",
  "gene_name": "U5 small nuclear ribonucleoprotein TSSC4",
  "gene": "UniProtKB:Q9Y5U2",
  "term_id": "GO:0140313"
}